{
  "term_label": "Unknown biological process",
  "gene_name": "Olfactory receptor 6M1",
  "gene_symbol": "OR6M1",
  "term_id": "UNKNOWN:0002",
  "gene": "UniProtKB:Q8NGM8"
}